{
  "gene_symbol": "ITGA10",
  "term_id": "GO:0034680",
  "gene": "UniProtKB:O75578",
  "term_label": "integrin alpha10-beta1 complex",
  "gene_name": "Integrin alpha-10"
}